{
  "gene": "UniProtKB:Q86W26",
  "term_label": "regulation of inflammatory response",
  "gene_name": "NACHT, LRR and PYD domains-containing protein 10",
  "gene_symbol": "NLRP10",
  "term_id": "GO:0050727"
}